{
  "term_label": "Unknown biological process",
  "gene": "UniProtKB:P60370",
  "gene_symbol": "KRTAP10-5",
  "term_id": "UNKNOWN:0002",
  "gene_name": "Keratin-associated protein 10-5"
}